cornified envelope [GO:0001533] (cellular component) Definition: A type of plasma membrane that has been modified through addition of distinct intracellular and extracellular components, including ceramide, found in cornifying epithelial cells (corneocytes). References: PMID:11112355, PMID:11590230, PMID:15803139 Sources: GOC:add Relationships: is_a plasma membrane [GO:0005886]